{
  "term_label": "Unknown biological process",
  "gene_symbol": "GAL3ST3",
  "gene": "UniProtKB:Q96A11",
  "term_id": "UNKNOWN:0002",
  "gene_name": "Galactose-3-O-sulfotransferase 3"
}